{
  "term_label": "Unknown cellular component",
  "gene": "UniProtKB:P57772",
  "gene_name": "Selenocysteine-specific elongation factor",
  "term_id": "UNKNOWN:0003",
  "gene_symbol": "EEFSEC"
}